{
  "term_label": "cell adhesion",
  "term_id": "GO:0007155",
  "gene_symbol": "CLDN6",
  "gene": "UniProtKB:P56747",
  "gene_name": "Claudin-6"
}